{
  "gene_symbol": "CCL18",
  "gene_name": "C-C motif chemokine 18",
  "term_id": "GO:0030335",
  "term_label": "positive regulation of cell migration",
  "gene": "UniProtKB:P55774"
}